protein targeting [GO:0006605] (biological process) Definition: The process of targeting specific proteins to particular regions of the cell, typically membrane-bounded subcellular organelles. Usually requires an organelle specific protein sequence motif. Also known as: protein sorting along secretory pathway, nascent polypeptide association Relationships: is a type of establishment of protein localization [GO:0045184] Regulation: regulated by GO:1903533 Subtypes: GO:0006612, GO:0006623, GO:0006625, protein targeting to mitochondrion [GO:0006626], protein targeting to chloroplast [GO:0045036], protein targeting to ER [GO:0045047], protein targeting to Golgi apparatus [GO:0140450] Sources: GOC:ma